{
  "gene": "UniProtKB:A6NCL1",
  "term_id": "GO:0005634",
  "term_label": "nucleus",
  "gene_symbol": "GMNC",
  "gene_name": "Geminin coiled-coil domain-containing protein 1"
}